{
  "term_label": "heat shock protein binding",
  "term_id": "GO:0031072",
  "gene_symbol": "CDC37",
  "gene": "UniProtKB:Q16543",
  "gene_name": "Hsp90 co-chaperone Cdc37"
}